{
  "gene_symbol": "FADS3",
  "gene": "UniProtKB:Q9Y5Q0",
  "gene_name": "Fatty acid desaturase 3",
  "term_label": "lipid metabolic process",
  "term_id": "GO:0006629"
}